{
  "term_id": "GO:0042995",
  "term_label": "cell projection",
  "gene": "UniProtKB:Q8NDC4",
  "gene_name": "MORN repeat-containing protein 4",
  "gene_symbol": "MORN4"
}